{
  "gene": "UniProtKB:O75771",
  "gene_name": "DNA repair protein RAD51 homolog 4",
  "term_label": "DNA strand invasion",
  "gene_symbol": "RAD51D",
  "term_id": "GO:0042148"
}